{
  "term_id": "UNKNOWN:0003",
  "gene_name": "Sodium_hydrogen exchanger 8",
  "gene_symbol": "SLC9A8",
  "gene": "UniProtKB:Q9Y2E8",
  "term_label": "Unknown cellular component"
}